{
  "gene_name": "Serine_threonine-protein kinase 3",
  "term_id": "GO:0035556",
  "term_label": "intracellular signal transduction",
  "gene_symbol": "STK3",
  "gene": "UniProtKB:Q13188"
}